{
  "term_id": "GO:0005085",
  "gene_name": "Rap guanine nucleotide exchange factor 3",
  "gene": "UniProtKB:O95398",
  "gene_symbol": "RAPGEF3",
  "term_label": "guanyl-nucleotide exchange factor activity"
}